{
  "term_id": "GO:0043236",
  "gene_symbol": "DAG1",
  "term_label": "laminin binding",
  "gene_name": "Dystroglycan 1",
  "gene": "UniProtKB:Q14118"
}